{
  "gene": "UniProtKB:Q6NS38",
  "term_label": "broad specificity oxidative DNA demethylase activity",
  "term_id": "GO:0035516",
  "gene_name": "DNA oxidative demethylase ALKBH2",
  "gene_symbol": "ALKBH2"
}